{
  "gene_name": "MMS19 nucleotide excision repair protein homolog",
  "term_id": "GO:0097361",
  "gene": "UniProtKB:Q96T76",
  "gene_symbol": "MMS19",
  "term_label": "cytosolic [4Fe-4S] assembly targeting complex"
}